{
  "gene": "UniProtKB:P41595",
  "gene_symbol": "HTR2B",
  "gene_name": "5-hydroxytryptamine receptor 2B",
  "term_label": "G protein-coupled receptor signaling pathway, coupled to cyclic nucleotide second messenger",
  "term_id": "GO:0007187"
}